{
  "gene_name": "Bcl-2-associated transcription factor 1",
  "gene_symbol": "BCLAF1",
  "term_id": "GO:0003712",
  "term_label": "transcription coregulator activity",
  "gene": "UniProtKB:Q9NYF8"
}